mitotic septin complex [GO:0032151] (cellular component) Definition: A heterooligomeric septin complex that acts during mitotic cell division. References: PMID:16009555 Sources: GOC:krc Relationships: is a type of GO:0031105